{
  "term_label": "nucleus",
  "term_id": "GO:0005634",
  "gene_symbol": "KHDC4",
  "gene_name": "KH homology domain-containing protein 4",
  "gene": "UniProtKB:Q7Z7F0"
}